{
  "gene_name": "Cytochrome P450 2F1",
  "gene_symbol": "CYP2F1",
  "term_label": "arachidonate epoxygenase activity",
  "gene": "UniProtKB:P24903",
  "term_id": "GO:0008392"
}